chloroplast outer membrane [GO:0009707] (CC) Relationships: is a type of plastid outer membrane [GO:0009527]; is a type of chloroplast membrane [GO:0031969] Also known as: chloroplast outer envelope Definition: The outer, i.e. cytoplasm-facing, lipid bilayer of the chloroplast envelope. Sources: GOC:tb